{
  "term_id": "GO:0008543",
  "term_label": "fibroblast growth factor receptor signaling pathway",
  "gene_name": "Fibroblast growth factor 10",
  "gene": "UniProtKB:O15520",
  "gene_symbol": "FGF10"
}